{
  "gene_name": "Sodium bicarbonate cotransporter 3",
  "term_id": "GO:0016323",
  "gene": "UniProtKB:Q9Y6M7",
  "term_label": "basolateral plasma membrane",
  "gene_symbol": "SLC4A7"
}